protein kinase C deactivation [GO:0042313] (biological process) Also known as: PKC deactivation Relationships: is a type of regulation of G protein-coupled receptor signaling pathway [GO:0008277] Sources: GOC:bf Definition: Any process resulting in the inhibition or termination of the activity of protein kinase C.